negative regulation of vascular associated smooth muscle cell apoptotic process [GO:1905460] (biological process) References: PMID:26493107 Sources: GOC:BHF, GOC:BHF_miRNA, GOC:TermGenie, GOC:rph, GO_REF:0000058 Also known as: down regulation of VSMC apoptotic process, down regulation of vascular associated smooth muscle cell apoptotic process, down regulation of vascular smooth muscle cell apoptotic process, down-regulation of VSMC apoptotic process, down-regulation of vascular associated smooth muscle cell apoptotic process, down-regulation of vascular smooth muscle cell apoptotic process, downregulation of VSMC apoptotic process, downregulation of vascular associated smooth muscle cell apoptotic process, downregulation of vascular smooth muscle cell apoptotic process, negative regulation of VSMC apoptotic process, negative regulation of vascular smooth muscle cell apoptotic process, down regulation of VSMC apoptosis, down regulation of vascular associated smooth muscle cell apoptosis, down regulation of vascular smooth muscle cell apoptosis, down-regulation of VSMC apoptosis, down-regulation of vascular associated smooth muscle cell apoptosis, down-regulation of vascular smooth muscle cell apoptosis, downregulation of VSMC apoptosis, downregulation of vascular associated smooth muscle cell apoptosis, downregulation of vascular smooth muscle cell apoptosis, inhibition of VSMC apoptosis, inhibition of VSMC apoptotic process, inhibition of vascular associated smooth muscle cell apoptosis, inhibition of vascular associated smooth muscle cell apoptotic process, inhibition of vascular smooth muscle cell apoptosis, inhibition of vascular smooth muscle cell apoptotic process, negative regulation of VSMC apoptosis, negative regulation of vascular associated smooth muscle cell apoptosis, negative regulation of vascular smooth muscle cell apoptosis Relationships: is a type of GO:0034392; is a type of regulation of vascular associated smooth muscle cell apoptotic process [GO:1905459]; negatively regulates GO:1905288 Definition: Any process that stops, prevents or reduces the frequency, rate or extent of vascular associated smooth muscle cell apoptotic process.